{
  "term_id": "UNKNOWN:0002",
  "term_label": "Unknown biological process",
  "gene": "UniProtKB:Q9UNP4",
  "gene_name": "Lactosylceramide alpha-2,3-sialyltransferase",
  "gene_symbol": "ST3GAL5"
}